{
  "gene_name": "BMP_retinoic acid-inducible neural-specific protein 2",
  "gene": "UniProtKB:Q9C0B6",
  "gene_symbol": "BRINP2",
  "term_label": "negative regulation of mitotic cell cycle",
  "term_id": "GO:0045930"
}